{
  "term_id": "UNKNOWN:0003",
  "term_label": "Unknown cellular component",
  "gene_symbol": "EIF5A2",
  "gene_name": "Eukaryotic translation initiation factor 5A-2",
  "gene": "UniProtKB:Q9GZV4"
}